{
  "gene": "UniProtKB:Q9Y5E8",
  "gene_symbol": "PCDHB15",
  "term_label": "cell adhesion molecule binding",
  "term_id": "GO:0050839",
  "gene_name": "Protocadherin beta-15"
}